negative regulation of programmed necrotic cell death [GO:0062099] (biological process) Subtypes: negative regulation of necroptotic process [GO:0060546] Definition: Any process that decreases the frequency, rate or extent of programmed necrotic cell death. References: PMID:27258785 Sources: GOC:aruk, GOC:rph Relationships: is a type of negative regulation of programmed cell death [GO:0043069]; is a type of regulation of programmed necrotic cell death [GO:0062098]; negatively regulates programmed necrotic cell death [GO:0097300]